GMP catabolic process to IMP [GO:0006201] (BP) Also known as: GMP breakdown to IMP, GMP degradation to IMP Definition: The chemical reactions and pathways resulting in the breakdown of guanosine monophosphate into other compounds, including inosine monophosphate. Relationships: is a type of GMP catabolic process [GO:0046038]; is a type of IMP metabolic process [GO:0046040] Sources: ISBN:0198506732